{
  "term_label": "protein serine/threonine kinase activity",
  "gene_symbol": "DAPK1",
  "gene_name": "Death-associated protein kinase 1",
  "term_id": "GO:0004674",
  "gene": "UniProtKB:P53355"
}